{
  "gene": "UniProtKB:P08134",
  "gene_symbol": "RHOC",
  "term_label": "plasma membrane",
  "term_id": "GO:0005886",
  "gene_name": "Rho-related GTP-binding protein RhoC"
}